{
  "gene_symbol": "F8A3",
  "term_id": "GO:0005769",
  "gene_name": "40-kDa huntingtin-associated protein",
  "term_label": "early endosome",
  "gene": "UniProtKB:P23610"
}